{
  "gene_symbol": "LMO2",
  "term_id": "GO:0005634",
  "gene_name": "Rhombotin-2",
  "term_label": "nucleus",
  "gene": "UniProtKB:P25791"
}